{
  "gene_name": "Pantothenate kinase 3",
  "gene": "UniProtKB:Q9H999",
  "gene_symbol": "PANK3",
  "term_id": "GO:0015937",
  "term_label": "coenzyme A biosynthetic process"
}